{
  "gene_name": "V-type proton ATPase subunit E 1",
  "term_id": "UNKNOWN:0002",
  "gene_symbol": "ATP6V1E1",
  "term_label": "Unknown biological process",
  "gene": "UniProtKB:P36543"
}